{
  "gene": "UniProtKB:Q9NZ08",
  "term_label": "Unknown cellular component",
  "gene_symbol": "ERAP1",
  "gene_name": "Endoplasmic reticulum aminopeptidase 1",
  "term_id": "UNKNOWN:0003"
}